negative regulation of serotonin biosynthetic process [GO:1905628] (biological process) Definition: Any process that stops, prevents or reduces the frequency, rate or extent of serotonin biosynthetic process. References: PMID:25642596 Sources: GOC:PARL, GOC:TermGenie, GOC:pad, GO_REF:0000058 Also known as: down regulation of serotonin anabolism, down regulation of serotonin biosynthesis, down regulation of serotonin biosynthetic process, down regulation of serotonin formation, down regulation of serotonin synthesis, down-regulation of serotonin anabolism, down-regulation of serotonin biosynthesis, down-regulation of serotonin biosynthetic process, down-regulation of serotonin formation, down-regulation of serotonin synthesis, downregulation of serotonin anabolism, downregulation of serotonin biosynthesis, downregulation of serotonin biosynthetic process, downregulation of serotonin formation, downregulation of serotonin synthesis, negative regulation of serotonin anabolism, negative regulation of serotonin biosynthesis, negative regulation of serotonin formation, negative regulation of serotonin synthesis, inhibition of serotonin anabolism, inhibition of serotonin biosynthesis, inhibition of serotonin biosynthetic process, inhibition of serotonin formation, inhibition of serotonin synthesis Relationships: is a type of negative regulation of biosynthetic process [GO:0009890]; is a type of GO:1905627; negatively regulates serotonin biosynthetic process [GO:0042427]